{
  "gene": "UniProtKB:P61296",
  "term_label": "DNA-binding transcription factor activity, RNA polymerase II-specific",
  "gene_symbol": "HAND2",
  "gene_name": "Heart- and neural crest derivatives-expressed protein 2",
  "term_id": "GO:0000981"
}